{
  "gene_name": "E3 ubiquitin-protein ligase HUWE1",
  "term_label": "nucleus",
  "gene_symbol": "HUWE1",
  "gene": "UniProtKB:Q7Z6Z7",
  "term_id": "GO:0005634"
}